{
  "gene_name": "Neuron-specific vesicular protein calcyon",
  "gene": "UniProtKB:Q9NYX4",
  "term_label": "clathrin light chain binding",
  "gene_symbol": "CALY",
  "term_id": "GO:0032051"
}